{
  "term_id": "UNKNOWN:0002",
  "gene_name": "Keratinocyte proline-rich protein",
  "gene": "UniProtKB:Q5T749",
  "term_label": "Unknown biological process",
  "gene_symbol": "KPRP"
}